raffinose alpha-galactosidase activity [GO:0052692] (molecular function) Definition: Catalysis of the reaction: raffinose + H2O = alpha-D-galactose + sucrose. References: PMID:20739305 Sources: RHEA:70275 Also known as: alkaline alpha-galactosidase activity, raffinose galactohydrolase activity, raffinose-specific alkaline alpha-galactosidase activity Relationships: is a type of GO:0004557